interleukin-10 receptor binding [GO:0005141] (molecular function) Also known as: IL-10, interleukin-10 receptor ligand Definition: Binding to an interleukin-10 receptor. Sources: GOC:ai Relationships: is a type of cytokine receptor binding [GO:0005126]; is_a growth factor receptor binding [GO:0070851]